{
  "gene_name": "RE1-silencing transcription factor",
  "gene_symbol": "REST",
  "term_label": "transcription cis-regulatory region binding",
  "term_id": "GO:0000976",
  "gene": "UniProtKB:Q13127"
}